endosome to lysosome transport via multivesicular body sorting pathway [GO:0032510] (biological process) Definition: The directed movement of substances from endosomes to lysosomes by a pathway in which molecules are sorted into multivesicular bodies, which then fuse with the lysosome. References: PMID:12461556, PMID:16689637 Sources: GOC:mah Also known as: endosome to lysosome transport via MVB sorting pathway Subtypes: late endosome to lysosome transport via multivesicular body sorting pathway [GO:0061764] Relationships: is a type of endosome to lysosome transport [GO:0008333]; is a type of GO:0032509